photoreceptor inner segment membrane [GO:0060342] (cellular component) Sources: GOC:dph Relationships: is a type of plasma membrane region [GO:0098590]; is part of photoreceptor inner segment [GO:0001917] Definition: The membrane surrounding the inner segment of a vertebrate photoreceptor. The photoreceptor inner segment contains mitochondria, ribosomes and membranes where opsin molecules are assembled and passed to be part of the outer segment discs.